pyruvate fermentation via PFL [GO:0044814] (biological process) References: PMID:19752030, PMID:2248795 Relationships: is a type of pyruvate fermentation [GO:0019660]; has part GO:0008861 Also known as: glycolytic fermentation via PFL pathway Definition: The anaerobic metabolic process in which pyruvate is converted to acetyl-CoA and formate by the action of pyruvate formate lyase (PFL), typically occurring in facultative anaerobic bacteria during mixed-acid fermentation.